{
  "gene_symbol": "SYT13",
  "term_id": "GO:0099502",
  "term_label": "calcium-dependent activation of synaptic vesicle fusion",
  "gene_name": "Synaptotagmin-13",
  "gene": "UniProtKB:Q7L8C5"
}